{
  "gene_symbol": "TSHR",
  "gene": "UniProtKB:P16473",
  "term_id": "GO:0007189",
  "term_label": "adenylate cyclase-activating G protein-coupled receptor signaling pathway",
  "gene_name": "Thyrotropin receptor"
}